{
  "term_id": "UNKNOWN:0003",
  "gene_symbol": "TPRX1",
  "term_label": "Unknown cellular component",
  "gene": "UniProtKB:Q8N7U7",
  "gene_name": "Tetra-peptide repeat homeobox protein 1"
}